{
  "term_id": "GO:0042054",
  "gene": "UniProtKB:Q96LA8",
  "gene_name": "Protein arginine N-methyltransferase 6",
  "term_label": "histone methyltransferase activity",
  "gene_symbol": "PRMT6"
}